{
  "gene": "UniProtKB:Q9BVP2",
  "term_label": "Unknown molecular function",
  "gene_name": "Guanine nucleotide-binding protein-like 3",
  "term_id": "UNKNOWN:0001",
  "gene_symbol": "GNL3"
}